{
  "term_label": "translation initiation factor binding",
  "gene_symbol": "EIF2B5",
  "term_id": "GO:0031369",
  "gene": "UniProtKB:Q13144",
  "gene_name": "Translation initiation factor eIF-2B subunit epsilon"
}